{
  "gene": "UniProtKB:A0A0B4J1Z2",
  "term_id": "GO:0019814",
  "gene_symbol": "IGKV1D-43",
  "term_label": "immunoglobulin complex",
  "gene_name": "Immunoglobulin kappa variable 1D-43"
}